ESCRT III complex assembly [GO:1904902] (biological process) Definition: The aggregation, arrangement and bonding together of a set of components to form an ESCRT III complex. Also known as: ESCRT III complex formation Relationships: is a type of GO:1904895 References: PMID:20588296 Sources: GOC:PARL, GOC:TermGenie, GOC:pad, GO_REF:0000079